cellular response to parathyroid hormone stimulus [GO:0071374] (biological process) Sources: GOC:mah Relationships: is a type of cellular response to hormone stimulus [GO:0032870]; is a type of response to parathyroid hormone [GO:0071107] Definition: Any process that results in a change in state or activity of a cell (in terms of movement, secretion, enzyme production, gene expression, etc.) as a result of a parathyroid hormone stimulus.